interleukin-35 receptor activity [GO:0070747] (molecular function) Sources: GOC:add, GOC:signaling Definition: Combining with interleukin-35 and transmitting the signal from one side of the membrane to the other to initiate a change in cell activity. Also known as: IL-35 receptor activity, IL-35R Relationships: is a type of cytokine receptor activity [GO:0004896]; is part of GO:0070757; has part interleukin-35 binding [GO:0070746]